fruit ripening, climacteric [GO:0009836] (biological process) Sources: GOC:lr, ISBN:0521587840 Relationships: is a type of fruit ripening [GO:0009835] Definition: A fruit ripening process that involves a burst of respiration and ethylene (ethene) evolution at the onset.